{
  "term_id": "GO:0031084",
  "gene_symbol": "HPS3",
  "gene_name": "BLOC-2 complex member HPS3",
  "term_label": "BLOC-2 complex",
  "gene": "UniProtKB:Q969F9"
}